{
  "gene_symbol": "POLR2C",
  "gene": "UniProtKB:P19387",
  "gene_name": "DNA-directed RNA polymerase II subunit RPB3",
  "term_label": "RNA polymerase II, core complex",
  "term_id": "GO:0005665"
}